{
  "term_id": "GO:0031545",
  "gene": "UniProtKB:Q9H6Z9",
  "gene_symbol": "EGLN3",
  "gene_name": "Prolyl hydroxylase EGLN3",
  "term_label": "peptidyl-proline 4-dioxygenase activity"
}